{
  "gene": "UniProtKB:Q96JQ2",
  "term_label": "nuclear outer membrane",
  "term_id": "GO:0005640",
  "gene_name": "Calmin",
  "gene_symbol": "CLMN"
}